histone H3K14ub reader activity [GO:0140258] (molecular function) Note: Comment: Note that the residue position corresponds to the canonical human H3 histone (UniProtKB:P84243); this residue is conserved across all eukaryotes. Residue 1 is the first residue following removal of the initiating Methionine (Met). Note that each histone is encoded by multiple genes, and sequences may vary across different genes within an organism. Also known as: H3-K14ub reader activity, H3K14ub modified histone binding Relationships: is a type of histone H3 reader activity [GO:0140006] References: PMID:29053958, PMID:34524082 Definition: A histone reader that recognizes a histone H3 ubiquitinated at lysine 14.